cellular response to lipoprotein particle stimulus [GO:0071402] (biological process) Definition: Any process that results in a change in state or activity of a cell (in terms of movement, secretion, enzyme production, gene expression, etc.) as a result of a lipoprotein particle stimulus. Relationships: is a type of GO:0051716 Subtypes: cellular response to high density lipoprotein particle stimulus [GO:0071403], cellular response to low-density lipoprotein particle stimulus [GO:0071404], GO:0090731 Sources: GOC:mah